{
  "term_label": "GTPase activator activity",
  "gene_symbol": "ARFGAP2",
  "term_id": "GO:0005096",
  "gene_name": "ADP-ribosylation factor GTPase-activating protein 2",
  "gene": "UniProtKB:Q8N6H7"
}